{
  "gene_symbol": "ZNF124",
  "term_id": "GO:0005634",
  "gene_name": "Zinc finger protein 124",
  "gene": "UniProtKB:Q15973",
  "term_label": "nucleus"
}